{
  "term_id": "UNKNOWN:0003",
  "gene": "UniProtKB:Q15777",
  "term_label": "Unknown cellular component",
  "gene_name": "Metallophosphoesterase MPPED2",
  "gene_symbol": "MPPED2"
}